{
  "gene_symbol": "SCNN1B",
  "gene": "UniProtKB:P51168",
  "term_label": "sodium channel complex",
  "gene_name": "Amiloride-sensitive sodium channel subunit beta",
  "term_id": "GO:0034706"
}